chondroitin hydrolase activity [GO:0052757] (molecular function) Relationships: is a type of GO:0033931 Definition: Catalysis of the hydrolysis of hexosaminic linkages in chondroitin, a linear polymer structure composed of the repeating disaccharide unit [->4)-D-glucuronic acid-(1->3)-N-acetyl-D-galactosamine-(1-], also written as [->4GlcUA1->3GalNAc1-]. Also known as: chondroitin endo-beta-galactosaminidase activity References: PMID:18390555 Sources: GOC:mengo_curators